{
  "gene_symbol": "UPK3BL1",
  "term_id": "UNKNOWN:0002",
  "gene": "UniProtKB:B0FP48",
  "term_label": "Unknown biological process",
  "gene_name": "Uroplakin-3b-like protein 1"
}